{
  "gene_symbol": "SESN3",
  "term_id": "GO:1904262",
  "gene_name": "Sestrin-3",
  "gene": "UniProtKB:P58005",
  "term_label": "negative regulation of TORC1 signaling"
}